{
  "term_id": "UNKNOWN:0003",
  "gene": "UniProtKB:Q5T9S5",
  "term_label": "Unknown cellular component",
  "gene_symbol": "CCDC18",
  "gene_name": "Coiled-coil domain-containing protein 18"
}